{
  "gene_symbol": "GPHA2",
  "gene_name": "Glycoprotein hormone alpha-2",
  "term_label": "extracellular space",
  "term_id": "GO:0005615",
  "gene": "UniProtKB:Q96T91"
}